{
  "term_label": "plasma membrane",
  "gene": "UniProtKB:O95297",
  "term_id": "GO:0005886",
  "gene_symbol": "MPZL1",
  "gene_name": "Myelin protein zero-like protein 1"
}